{
  "gene": "UniProtKB:O14672",
  "term_label": "metalloendopeptidase activity involved in amyloid precursor protein catabolic process",
  "gene_symbol": "ADAM10",
  "term_id": "GO:1902945",
  "gene_name": "Disintegrin and metalloproteinase domain-containing protein 10"
}